Derlin-1-VIMP complex [GO:0036502] (CC) References: PMID:15215856, PMID:16186510 Sources: GOC:PARL, GOC:bf Definition: A protein complex containing, in mammals, Derlin-1 and VCP-interacting membrane protein (VIMP). The complex links the p97/VCP-containing ATPase complex with Derlin-1 during translocation of protein substrates from the endoplasmic reticulum to the cytosol for degradation by the cytosolic proteasome. Also known as: Derlin-1/VIMP complex Relationships: is a type of membrane protein complex [GO:0098796]; is a type of endoplasmic reticulum protein-containing complex [GO:0140534]; is part of endoplasmic reticulum membrane [GO:0005789]